{
  "term_label": "immunoglobulin complex",
  "gene_symbol": "IGLV1-40",
  "gene": "UniProtKB:P01703",
  "gene_name": "Immunoglobulin lambda variable 1-40",
  "term_id": "GO:0019814"
}